proline import across plasma membrane [GO:1905647] (biological process) References: PMID:24344203 Sources: GOC:TermGenie, GO_REF:0000075 Definition: The directed movement of proline from outside of a cell into the cytoplasmic compartment. Subtypes: L-proline import across plasma membrane [GO:1904271] Regulation: RO_0002211 by regulation of proline import across plasma membrane [GO:1902834]; negatively regulated by negative regulation of proline import across plasma membrane [GO:1902835]; positively regulated by GO:1902836 Also known as: proline import into cell Relationships: is a type of GO:0035524; is a type of amino acid import across plasma membrane [GO:0089718]